cellular response to calcium ion starvation [GO:0072732] (biological process) Sources: GOC:mah Definition: Any process that results in a change in state or activity of a cell (in terms of movement, secretion, enzyme production, gene expression, etc.) as a result of deprivation of calcium ions. Relationships: is a type of GO:0009267 Also known as: cellular response to calcium starvation